{
  "gene_name": "Putative ankyrin repeat domain-containing protein 20A12 pseudogene",
  "gene": "UniProtKB:Q8NF67",
  "term_id": "UNKNOWN:0001",
  "term_label": "Unknown molecular function",
  "gene_symbol": "ANKRD20A12P"
}